regulation of anthocyanin catabolic process [GO:1900000] (biological process) Relationships: is a type of regulation of catabolic process [GO:0009894]; is a type of GO:0031537; regulates anthocyanin-containing compound catabolic process [GO:0046284] Also known as: regulation of anthocyanin breakdown, regulation of anthocyanin catabolism, regulation of anthocyanin degradation Definition: Any process that modulates the frequency, rate or extent of anthocyanin catabolic process. Sources: GOC:TermGenie Subtypes: negative regulation of anthocyanin catabolic process [GO:1900001], GO:1900002